{
  "gene": "UniProtKB:P30048",
  "term_label": "hydrogen peroxide catabolic process",
  "gene_symbol": "PRDX3",
  "gene_name": "Thioredoxin-dependent peroxide reductase, mitochondrial",
  "term_id": "GO:0042744"
}